{
  "term_id": "GO:0000978",
  "gene_name": "Endoplasmic reticulum membrane sensor NFE2L1",
  "gene_symbol": "NFE2L1",
  "term_label": "RNA polymerase II cis-regulatory region sequence-specific DNA binding",
  "gene": "UniProtKB:Q14494"
}